response to photoperiod, blue light [GO:0009906] (biological process) Definition: Any process that results in a change in state or activity of a cell or an organism (in terms of movement, secretion, enzyme production, gene expression, etc.) as a result of the detection of a blue light photoperiod stimulus. Blue light is electromagnetic radiation with a wavelength of between 440 and 500nm. Sources: GOC:go_curators, GOC:mtg_far_red Relationships: is a type of response to blue light [GO:0009637]; is a type of photoperiodism [GO:0009648]